{
  "term_label": "protein import into nucleus",
  "term_id": "GO:0006606",
  "gene_name": "Protein FAM53B",
  "gene_symbol": "FAM53B",
  "gene": "UniProtKB:Q14153"
}